{
  "gene_name": "Myosin-10",
  "term_id": "GO:0000281",
  "gene_symbol": "MYH10",
  "gene": "UniProtKB:P35580",
  "term_label": "mitotic cytokinesis"
}